{
  "gene_symbol": "TRIM39",
  "gene": "UniProtKB:Q9HCM9",
  "term_label": "cytosol",
  "gene_name": "E3 ubiquitin-protein ligase TRIM39",
  "term_id": "GO:0005829"
}